{
  "gene_name": "Forkhead box protein D2",
  "term_id": "GO:0006357",
  "term_label": "regulation of transcription by RNA polymerase II",
  "gene_symbol": "FOXD2",
  "gene": "UniProtKB:O60548"
}